embryonic epithelial tube formation [GO:0001838] (biological process) Definition: The morphogenesis of an embryonic epithelium into a tube-shaped structure. Sources: GOC:dph, ISBN:0824072820 Relationships: is a type of epithelial tube formation [GO:0072175]; is part of morphogenesis of embryonic epithelium [GO:0016331] Subtypes: neural tube formation [GO:0001841], embryonic heart tube formation [GO:0003144], GO:0014020, secondary neural tube formation [GO:0014021], nephron tubule formation [GO:0072079]